temporomandibular joint articular cartilage development [GO:0061976] (biological process) Subtypes: mandibular condyle articular cartilage development [GO:0061978] Relationships: is a type of articular cartilage development [GO:0061975] References: PMID:20679519 Definition: The process whose specific outcome is the progression of temporomandibular joint articular cartilage over time, from its formation to the mature structure.